{
  "term_id": "GO:0005739",
  "gene_name": "Protein NipSnap homolog 3A",
  "term_label": "mitochondrion",
  "gene": "UniProtKB:Q9UFN0",
  "gene_symbol": "NIPSNAP3A"
}